{
  "term_id": "GO:0005829",
  "gene_symbol": "DPH3P1",
  "term_label": "cytosol",
  "gene_name": "Putative DPH3 homolog B",
  "gene": "UniProtKB:Q9H4G8"
}